dormancy maintenance of symbiont in host [GO:0085015] (BP) Definition: Any process in which a dormant state is maintained by the symbiont within the host organism. Also known as: NRP, non-replicating persistence Sources: GOC:jl Relationships: is a type of dormancy process [GO:0022611]; is a type of development of symbiont in host [GO:0044114]